{
  "gene_symbol": "TIMD4",
  "term_id": "UNKNOWN:0003",
  "gene_name": "T-cell immunoglobulin and mucin domain-containing protein 4",
  "term_label": "Unknown cellular component",
  "gene": "UniProtKB:Q96H15"
}